{
  "gene_name": "Hypermethylated in cancer 1 protein",
  "gene": "UniProtKB:Q14526",
  "gene_symbol": "HIC1",
  "term_label": "regulation of transcription by RNA polymerase II",
  "term_id": "GO:0006357"
}